{
  "term_label": "cytoplasm",
  "term_id": "GO:0005737",
  "gene_symbol": "SPA17",
  "gene": "UniProtKB:Q15506",
  "gene_name": "Sperm surface protein Sp17"
}